cadmium ion transport [GO:0015691] (biological process) Relationships: is a type of transition metal ion transport [GO:0000041] Also known as: cadmium transport Sources: GOC:ai Subtypes: cadmium ion transmembrane transport [GO:0070574] Definition: The directed movement of cadmium (Cd) ions into, out of or within a cell, or between cells, by means of some agent such as a transporter or pore.